{
  "term_label": "Seh1-associated complex",
  "gene_name": "Nucleoporin SEH1",
  "gene": "UniProtKB:Q96EE3",
  "term_id": "GO:0035859",
  "gene_symbol": "SEH1L"
}